{
  "term_id": "UNKNOWN:0003",
  "gene_name": "Cilia- and flagella-associated protein 54",
  "gene": "UniProtKB:Q96N23",
  "term_label": "Unknown cellular component",
  "gene_symbol": "CFAP54"
}